negative regulation of peptidoglycan recognition protein signaling pathway [GO:0061060] (biological process) Also known as: negative regulation of peptidoglycan recognition protein signalling pathway Definition: Any process that decreases the rate, frequency, or extent of the peptidoglycan recognition protein signaling pathway. Sources: GOC:dph Relationships: is a type of GO:0002683; is a type of negative regulation of signal transduction [GO:0009968]; is a type of regulation of peptidoglycan recognition protein signaling pathway [GO:0061058]; is a type of GO:1900425; negatively regulates peptidoglycan recognition protein signaling pathway [GO:0061057]